atrioventricular node development [GO:0003162] (biological process) Relationships: is a type of cardiac muscle tissue development [GO:0048738]; is part of GO:0003161 Definition: The process whose specific outcome is the progression of the atrioventricular (AV) node over time, from its formation to the mature structure. The AV node is part of the cardiac conduction system that controls the timing of ventricle contraction by receiving electrical signals from the sinoatrial (SA) node and relaying them to the His-Purkinje system. Also known as: AV node development Sources: GOC:mtg_heart